maintenance of seed dormancy [GO:0010231] (biological process) Subtypes: maintenance of seed dormancy by absisic acid [GO:0098755] References: PMID:9580097 Sources: ISBN:9781405139830 Definition: Any process that maintains a seed in a dormant state. Relationships: is a type of GO:0010162; is a type of maintenance of dormancy [GO:0097437]